rRNA methylation [GO:0031167] (biological process) Definition: The posttranscriptional addition of methyl groups to specific residues in an rRNA molecule. Sources: GOC:mah Relationships: is a type of GO:0000154; is a type of RNA methylation [GO:0001510] Subtypes: GO:0000451, rRNA base methylation [GO:0070475]